{
  "gene_symbol": "AURKB",
  "gene": "UniProtKB:Q96GD4",
  "term_id": "GO:0000922",
  "gene_name": "Aurora kinase B",
  "term_label": "spindle pole"
}